negative regulation of leukocyte tethering or rolling [GO:1903237] (BP) Also known as: down regulation of leukocyte tethering or rolling, down-regulation of leukocyte tethering or rolling, downregulation of leukocyte tethering or rolling, inhibition of leukocyte tethering or rolling References: PMID:18308860 Sources: GOC:TermGenie, GOC:als, GO_REF:0000058 Definition: Any process that stops, prevents or reduces the frequency, rate or extent of leukocyte tethering or rolling. Relationships: is a type of negative regulation of cellular extravasation [GO:0002692]; is a type of regulation of leukocyte tethering or rolling [GO:1903236]; is a type of negative regulation of leukocyte adhesion to vascular endothelial cell [GO:1904995]; negatively regulates leukocyte tethering or rolling [GO:0050901]